{
  "term_id": "GO:0061685",
  "term_label": "diphthine methylesterase activity",
  "gene_symbol": "DPH7",
  "gene": "UniProtKB:Q9BTV6",
  "gene_name": "Diphthine methyltransferase"
}